alpha3-beta1 integrin-basigin complex [GO:0071080] (cellular component) Relationships: is a type of plasma membrane protein complex [GO:0098797] Also known as: ITGA3-ITGB1-BSG complex Definition: A protein complex that consists of an alpha3-beta1 integrin complex bound to the cell surface protein basigin. References: PMID:9360995